{
  "term_id": "GO:0000350",
  "term_label": "generation of catalytic spliceosome for second transesterification step",
  "gene_name": "Pre-mRNA-splicing factor ISY1 homolog",
  "gene_symbol": "ISY1",
  "gene": "UniProtKB:Q9ULR0"
}